{
  "gene": "UniProtKB:Q07021",
  "term_label": "nucleus",
  "gene_name": "Complement component 1 Q subcomponent-binding protein, mitochondrial",
  "gene_symbol": "C1QBP",
  "term_id": "GO:0005634"
}